cell proliferation in external granule layer [GO:0021924] (biological process) Relationships: is a type of cell proliferation in hindbrain [GO:0021534] Definition: The multiplication or reproduction of neuroblasts resulting in the expansion of a cell population in the external granule layer of the hindbrain. The external granule layer is the layer that originates from the rostral half of the rhombic lip in the first rhombomere. References: PMID:15157725 Sources: GOC:cls, GOC:dgh, GOC:dph, GOC:jid, GO_REF:0000021 Subtypes: cerebellar granule cell precursor proliferation [GO:0021930], rostral hindbrain neuronal precursor cell proliferation [GO:0021931]